{
  "gene_name": "Ferritin heavy polypeptide-like 17",
  "term_id": "GO:0008198",
  "gene": "UniProtKB:Q9BXU8",
  "gene_symbol": "FTHL17",
  "term_label": "ferrous iron binding"
}